{
  "gene_name": "Olfactory receptor 5D16",
  "gene_symbol": "OR5D16",
  "term_label": "G protein-coupled receptor signaling pathway",
  "term_id": "GO:0007186",
  "gene": "UniProtKB:Q8NGK9"
}